hexitol biosynthetic process [GO:0019406] (biological process) Subtypes: sorbitol biosynthetic process [GO:0006061], galactitol biosynthetic process [GO:0019403], mannitol biosynthetic process [GO:0019593] Definition: The chemical reactions and pathways resulting in the formation of hexitols, any alditol with a chain of six carbon atoms in the molecule. Relationships: is a type of GO:0006059; is a type of alditol biosynthetic process [GO:0019401] Sources: ISBN:0198506732 Also known as: hexitol anabolism, hexitol biosynthesis, hexitol formation, hexitol synthesis